glial cell-derived neurotrophic factor receptor signaling pathway involved in ureteric bud formation [GO:2000701] (biological process) Relationships: is_a GO:0035860; is part of GO:0060676 Also known as: GDNF receptor signaling pathway of ureteric bud formation, glial cell derived neurotrophic factor receptor signaling pathway of ureteric bud formation, glial cell line-derived neurotrophic factor receptor signalling pathway of ureteric bud formation, glial cell-derived neurotrophic factor receptor signaling pathway of ureteric bud formation, glial cell-derived neurotrophic factor receptor signalling pathway of ureteric bud formation Sources: GOC:mtg_kidney_jan10, GOC:obol, GOC:yaf Definition: The series of molecular signals generated as a consequence of a glial cell-derived neurotrophic factor receptor binding to one of its physiological ligands that contributes to the formation of the ureteric bud from the Wolffian duct. Regulation: regulated by regulation of glial cell-derived neurotrophic factor receptor signaling pathway involved in ureteric bud formation [GO:2000733]; negatively regulated by negative regulation of glial cell-derived neurotrophic factor receptor signaling pathway involved in ureteric bud formation [GO:2000734]; positively regulated by positive regulation of glial cell-derived neurotrophic factor receptor signaling pathway involved in ureteric bud formation [GO:2000735]